{
  "gene_name": "C-C motif chemokine 22",
  "gene_symbol": "CCL22",
  "term_id": "GO:0006954",
  "term_label": "inflammatory response",
  "gene": "UniProtKB:O00626"
}